{
  "gene_name": "Protein WWC3",
  "term_id": "GO:0006355",
  "gene_symbol": "WWC3",
  "gene": "UniProtKB:Q9ULE0",
  "term_label": "regulation of DNA-templated transcription"
}